response to deep water [GO:0030912] (biological process) Sources: GOC:mah Definition: Any process that results in a change in state or activity of a cell or an organism (in terms of movement, secretion, enzyme production, gene expression, etc.) as a result of a deep water stimulus, being immersed in standing deep water throughout the life cycle. Relationships: is_a response to water [GO:0009415] Note: Note that this term should not be confused with 'response to flooding ; GO:0009413'; which refers to immersion in water on a shorter time scale.